{
  "term_id": "GO:0030182",
  "term_label": "neuron differentiation",
  "gene": "UniProtKB:Q71U36",
  "gene_name": "Tubulin alpha-1A chain",
  "gene_symbol": "TUBA1A"
}